{
  "gene_symbol": "SPAG5",
  "term_label": "Unknown biological process",
  "gene_name": "Sperm-associated antigen 5",
  "gene": "UniProtKB:Q96R06",
  "term_id": "UNKNOWN:0002"
}